CCR2 chemokine receptor binding [GO:0031727] (molecular function) Relationships: is a type of CCR chemokine receptor binding [GO:0048020] Also known as: monocyte chemoattractant protein 1 receptor binding, CCR2 chemokine receptor ligand Sources: GOC:mah, GOC:nln Definition: Binding to a CCR2 chemokine receptor.